{
  "gene_name": "Neprilysin",
  "term_label": "plasma membrane",
  "term_id": "GO:0005886",
  "gene_symbol": "MME",
  "gene": "UniProtKB:P08473"
}